CAAX-box protein maturation [GO:0080120] (biological process) Definition: A series of specific posttranslational modifications to the CAAX box region of CAAX box proteins. CAAX box proteins are eukaryotic proteins that contain a CAAX motif where the C is a cysteine, the two A residues are aliphatic amino acids and the X can be one of several amino acids. The CAAX-box proteins undergo three sequential, enzymatic, post-translational modifications essential to their targeting: First, the proteins are prenylated by one of two prenyltransferases called farnesyltransferase and geranylgeranyltransferase-I. Prenylation results in the covalent attachment of either farnesyl or geranylgeranyl isoprenoid groups to the cysteine in the CAAX box motif. Prenylation is followed by proteolytic removal of the last three amino acids of the protein (AAX). Finally, the newly exposed carboxylate group of the isoprenylcysteine is methylated by an ER-associated prenyl-dependent carboxylmethyltransferase. Also known as: CAAX-box protein processing, farnesylated protein maturation References: PMID:12039957, PMID:17114793, PMID:18641086 Relationships: is a type of GO:0051604; has part protein processing [GO:0016485]; has part GO:0018342